pollen germination [GO:0009846] (biological process) References: PMID:30669423 Sources: GOC:lr, ISBN:0943088399 Relationships: is_a GO:0032501; BFO_0000050 GO:0009856 Definition: The physiological and developmental changes that occur in a heterosporous plant pollen grain, beginning with hydration and terminating with the emergence of the pollen tube through the aperture.